{
  "term_id": "GO:0006357",
  "term_label": "regulation of transcription by RNA polymerase II",
  "gene_name": "Zinc finger protein 232",
  "gene_symbol": "ZNF232",
  "gene": "UniProtKB:Q9UNY5"
}